{
  "term_id": "UNKNOWN:0001",
  "gene": "UniProtKB:Q9NNX1",
  "gene_name": "Tuftelin",
  "term_label": "Unknown molecular function",
  "gene_symbol": "TUFT1"
}